{
  "term_label": "Unknown biological process",
  "term_id": "UNKNOWN:0002",
  "gene": "UniProtKB:E7EW31",
  "gene_name": "Proline-rich basic protein 1",
  "gene_symbol": "PROB1"
}